{
  "gene_symbol": "ZNF236",
  "term_label": "nucleus",
  "term_id": "GO:0005634",
  "gene": "UniProtKB:Q9UL36",
  "gene_name": "Zinc finger protein 236"
}